{
  "gene": "UniProtKB:Q9H6Z9",
  "gene_name": "Prolyl hydroxylase EGLN3",
  "gene_symbol": "EGLN3",
  "term_id": "GO:0043523",
  "term_label": "regulation of neuron apoptotic process"
}